{
  "gene": "UniProtKB:P62310",
  "gene_symbol": "LSM3",
  "gene_name": "U6 snRNA-associated Sm-like protein LSm3",
  "term_id": "GO:0046540",
  "term_label": "U4/U6 x U5 tri-snRNP complex"
}